GDP-mannose 6-dehydrogenase activity [GO:0047919] (molecular function) Sources: EC:1.1.1.132, RHEA:21728 Definition: Catalysis of the reaction: GDP-alpha-D-mannose + H2O + 2 NAD+ = GDP-D-mannuronate + 3 H+ + 2 NADH. Also known as: GDP mannose dehydrogenase activity, GDP-D-mannose:NAD+ 6-oxidoreductase activity, GDPmannose 6-dehydrogenase activity, guanosine diphospho-D-mannose dehydrogenase activity, guanosine diphosphomannose dehydrogenase activity Relationships: is a type of oxidoreductase activity, acting on the CH-OH group of donors, NAD or NADP as acceptor [GO:0016616]